{
  "term_id": "GO:0003729",
  "term_label": "mRNA binding",
  "gene_name": "Eukaryotic initiation factor 4A-III",
  "gene_symbol": "EIF4A3",
  "gene": "UniProtKB:P38919"
}